{
  "gene_symbol": "DIS3",
  "gene": "UniProtKB:Q9Y2L1",
  "gene_name": "Exosome complex exonuclease RRP44",
  "term_label": "cytoplasmic exosome (RNase complex)",
  "term_id": "GO:0000177"
}